prevention of polyspermy [GO:0060468] (biological process) Relationships: is a type of negative regulation of fertilization [GO:0060467]; is part of egg activation [GO:0007343] Definition: The negative regulation of fertilization process that takes place as part of egg activation, ensuring that only a single sperm fertilizes the egg. Also known as: negative regulation of fertilization involved in egg activation, polyspermy block Sources: GOC:dph